homeostasis of number of cells [GO:0048872] (biological process) Definition: Any biological process involved in the maintenance of the steady-state number of cells within a population of cells. Relationships: is_a multicellular organismal-level homeostasis [GO:0048871] Subtypes: leukocyte homeostasis [GO:0001776], myeloid cell homeostasis [GO:0002262], hepatocyte homeostasis [GO:0036333], epidermal stem cell homeostasis [GO:0036334], intestinal stem cell homeostasis [GO:0036335], GO:0048873, GO:0048874, hematopoietic stem cell homeostasis [GO:0061484], host-mediated modulation of oral microbiota composition [GO:0120332] Sources: GOC:isa_complete Also known as: cell population homeostasis, homeostasis of cell number